complement activation, GZMK pathway [GO:0160257] (biological process) Relationships: is a type of complement activation [GO:0006956]; is a type of innate immune response [GO:0045087] Definition: Any process involved in the activation of any of the steps of the granzyme K pathway of the complement cascade which allows for the direct killing of microbes and the regulation of other immune processes. References: PMID:39814882, PMID:39914456 Also known as: complement activation, granzyme K pathway